{
  "gene_symbol": "SYN2",
  "gene": "UniProtKB:Q92777",
  "term_label": "synapse organization",
  "gene_name": "Synapsin-2",
  "term_id": "GO:0050808"
}